positive regulation of filamentous growth of a population of unicellular organisms in response to starvation [GO:1900436] (biological process) Definition: Any process that activates or increases the frequency, rate or extent of filamentous growth of a population of unicellular organisms in response to starvation. Also known as: up regulation of filamentous growth of a population of unicellular organisms in response to starvation, up-regulation of filamentous growth of a population of unicellular organisms in response to starvation, upregulation of filamentous growth of a population of unicellular organisms in response to starvation, activation of filamentous growth of a population of unicellular organisms in response to starvation Sources: GOC:TermGenie, GOC:di Relationships: is_a GO:0032109; is a type of positive regulation of filamentous growth of a population of unicellular organisms [GO:1900430]; is a type of regulation of filamentous growth of a population of unicellular organisms in response to starvation [GO:1900434]; positively regulates filamentous growth of a population of unicellular organisms in response to starvation [GO:0036170]